{
  "term_id": "UNKNOWN:0001",
  "term_label": "Unknown molecular function",
  "gene": "UniProtKB:P21953",
  "gene_symbol": "BCKDHB",
  "gene_name": "2-oxoisovalerate dehydrogenase subunit beta, mitochondrial"
}